borate transport [GO:0046713] (BP) Definition: The directed movement of borate into, out of or within a cell, or between cells, by means of some agent such as a transporter or pore. Borate is the anion (BO3)3-; boron is a group 13 element, with properties which are borderline between metals and non-metals. References: PMID:21710975 Also known as: boron transport Relationships: is a type of inorganic anion transport [GO:0015698] Subtypes: borate transmembrane transport [GO:0035445]